extracellular organelle [GO:0043230] (cellular component) Relationships: is a type of organelle [GO:0043226]; BFO_0000050 extracellular region [GO:0005576] Subtypes: extracellular membraneless organelle [GO:0043264], GO:0065010 References: PMID:9914479 Sources: GOC:jl Definition: Organized structure of distinctive morphology and function, occurring outside the cell. Includes, for example, extracellular membrane vesicles (EMVs) and the cellulosomes of anaerobic bacteria and fungi.